{
  "term_label": "Unknown cellular component",
  "term_id": "UNKNOWN:0003",
  "gene_symbol": "GXYLT1",
  "gene_name": "Glucoside xylosyltransferase 1",
  "gene": "UniProtKB:Q4G148"
}